cytoplasmic side of plasma membrane [GO:0009898] (cellular component) Sources: GOC:dos, GOC:tb Also known as: juxtamembrane, internal leaflet of plasma membrane, internal side of plasma membrane Relationships: is a type of cytoplasmic side of membrane [GO:0098562]; is part of plasma membrane [GO:0005886] Subtypes: GO:0098592, cytoplasmic side of plasma membrane, cell tip [GO:0106186], cytoplasmic side of dendritic spine plasma membrane [GO:1990780] Definition: The leaflet the plasma membrane that faces the cytoplasm and any proteins embedded or anchored in it or attached to its surface.